{
  "gene_name": "Protein phosphatase 1 regulatory subunit 15B",
  "term_label": "response to endoplasmic reticulum stress",
  "term_id": "GO:0034976",
  "gene": "UniProtKB:Q5SWA1",
  "gene_symbol": "PPP1R15B"
}